tRNA folding [GO:0061818] (biological process) References: PMID:27849601 Sources: GOC:dph Definition: The process of assisting in the folding of tRNAs into the correct tertiary structure. Relationships: is a type of RNA folding [GO:0034337]